{
  "gene": "UniProtKB:Q14982",
  "term_id": "GO:0005886",
  "gene_name": "Opioid-binding protein_cell adhesion molecule",
  "term_label": "plasma membrane",
  "gene_symbol": "OPCML"
}